{
  "term_label": "regulation of cytokinesis",
  "gene": "UniProtKB:Q96GD4",
  "gene_name": "Aurora kinase B",
  "term_id": "GO:0032465",
  "gene_symbol": "AURKB"
}